ergothioneine catabolic process [GO:0052700] (biological process) Definition: The chemical reactions and pathways resulting in the breakdown of ergothioneine, a naturally occurring metabolite of histidine with antioxidant properties. Sources: Wikipedia:Ergothioneine Also known as: (2S)-3-(2-mercapto-1H-imidazol-5-yl)-2-(trimethylazaniumyl)propanoate catabolic process, 2-mercaptoergothioneine trimethylbetaine breakdown, 2-mercaptoergothioneine trimethylbetaine catabolic process, 2-mercaptoergothioneine trimethylbetaine catabolism, 2-mercaptoergothioneine trimethylbetaine degradation, ergothioneine breakdown, ergothioneine catabolism, ergothioneine degradation Relationships: is a type of sulfur amino acid catabolic process [GO:0000098]; is a type of amino-acid betaine catabolic process [GO:0006579]; is a type of GO:0052698; is a type of modified histidine catabolic process [GO:0052702]